{
  "gene_symbol": "ARL8B",
  "term_label": "lysosomal membrane",
  "gene": "UniProtKB:Q9NVJ2",
  "term_id": "GO:0005765",
  "gene_name": "ADP-ribosylation factor-like protein 8B"
}